sialate O-acetylesterase activity [GO:0001681] (molecular function) Also known as: N-acetylneuraminate acetyltransferase activity Relationships: is a type of acetylesterase activity [GO:0008126] References: PMID:1991039 Sources: EC:3.1.1.53 Subtypes: sialate 9-O-acetylesterase activity [GO:0106330], sialate 4-O-acetylesterase activity [GO:0106331] Definition: Catalysis of the reaction: N-acetyl-O-acetylneuraminate (free or glycosidically bound) + H2O = N-acetylneuraminate + acetate.